{
  "gene_symbol": "KCNE4",
  "gene_name": "Potassium voltage-gated channel subfamily E member 4",
  "term_label": "ventricular cardiac muscle cell action potential",
  "term_id": "GO:0086005",
  "gene": "UniProtKB:Q8WWG9"
}